{
  "term_id": "GO:0047035",
  "gene_symbol": "HSD17B2",
  "term_label": "testosterone dehydrogenase (NAD+) activity",
  "gene": "UniProtKB:P37059",
  "gene_name": "17-beta-hydroxysteroid dehydrogenase type 2"
}